{
  "gene_name": "Protein GOLM2",
  "gene_symbol": "GOLM2",
  "gene": "UniProtKB:Q6P4E1",
  "term_label": "Unknown cellular component",
  "term_id": "UNKNOWN:0003"
}